{
  "gene": "UniProtKB:A6NMK8",
  "gene_name": "Protein INSYN2B",
  "term_label": "Unknown biological process",
  "term_id": "UNKNOWN:0002",
  "gene_symbol": "INSYN2B"
}